formylmethionine deformylase activity [GO:0008463] (molecular function) Relationships: is a type of GO:0016811 Sources: EC:3.5.1.31, RHEA:17781 Definition: Catalysis of the reaction: N-formyl-L-methionine + H2O = L-methionine + formate. Also known as: N-formyl-L-methionine amidohydrolase activity